{
  "gene_symbol": "ZNF189",
  "gene": "UniProtKB:O75820",
  "term_id": "GO:0005634",
  "term_label": "nucleus",
  "gene_name": "Zinc finger protein 189"
}